polyamine:proton antiporter activity [GO:0015312] (MF) Sources: TC:2.A.1.2.16 Definition: Enables the transfer of a solute or solutes from one side of a membrane to the other according to the reaction: H+(out) + polyamine(in) = H+(in) + polyamine(out). Also known as: polyamine:hydrogen antiporter activity Relationships: is a type of GO:0015078; is a type of polyamine transmembrane transporter activity [GO:0015203]; is a type of antiporter activity [GO:0015297]